{
  "gene_name": "Immunoglobulin lambda-like polypeptide 5",
  "gene_symbol": "IGLL5",
  "term_id": "GO:0016064",
  "term_label": "immunoglobulin mediated immune response",
  "gene": "UniProtKB:B9A064"
}